{
  "term_label": "Unknown biological process",
  "gene": "UniProtKB:Q8WVB3",
  "gene_name": "Hexosaminidase D",
  "gene_symbol": "HEXD",
  "term_id": "UNKNOWN:0002"
}